{
  "gene": "UniProtKB:Q96HE8",
  "term_id": "GO:0035869",
  "term_label": "ciliary transition zone",
  "gene_name": "Transmembrane protein 80",
  "gene_symbol": "TMEM80"
}